positive regulation of heart rate by neuronal epinephrine [GO:0003112] (biological process) Definition: The process in which the secretion of epinephrine from nerve endings increases the rate of heart muscle contraction. Also known as: positive regulation of heart rate by neuronal adrenaline Sources: GOC:mtg_cardio Relationships: is a type of positive regulation of heart rate by epinephrine [GO:0003065]